{
  "gene": "UniProtKB:Q9P2S2",
  "term_id": "GO:0004888",
  "term_label": "transmembrane signaling receptor activity",
  "gene_symbol": "NRXN2",
  "gene_name": "Neurexin-2"
}